{
  "gene_name": "Uncharacterized protein C18orf63",
  "term_id": "UNKNOWN:0003",
  "term_label": "Unknown cellular component",
  "gene": "UniProtKB:Q68DL7",
  "gene_symbol": "C18orf63"
}